{
  "term_label": "Unknown cellular component",
  "gene_symbol": "TMEM71",
  "gene": "UniProtKB:Q6P5X7",
  "term_id": "UNKNOWN:0003",
  "gene_name": "Transmembrane protein 71"
}